{
  "gene": "UniProtKB:P61952",
  "term_id": "GO:0007186",
  "gene_symbol": "GNG11",
  "gene_name": "Guanine nucleotide-binding protein G(I)_G(S)_G(O) subunit gamma-11",
  "term_label": "G protein-coupled receptor signaling pathway"
}